{
  "gene": "UniProtKB:Q6PEY2",
  "gene_name": "Tubulin alpha-3E chain",
  "term_label": "mitotic cell cycle",
  "term_id": "GO:0000278",
  "gene_symbol": "TUBA3E"
}